{
  "term_label": "homologous chromosome segregation",
  "gene_symbol": "PTTG2",
  "gene": "UniProtKB:Q9NZH5",
  "term_id": "GO:0045143",
  "gene_name": "Securin-2"
}